{
  "gene": "UniProtKB:Q1A5X6",
  "gene_name": "IQ domain-containing protein J",
  "term_label": "Unknown molecular function",
  "gene_symbol": "IQCJ",
  "term_id": "UNKNOWN:0001"
}